{
  "gene": "UniProtKB:Q13326",
  "term_label": "Unknown molecular function",
  "gene_name": "Gamma-sarcoglycan",
  "term_id": "UNKNOWN:0001",
  "gene_symbol": "SGCG"
}